{
  "gene": "UniProtKB:Q9H6K1",
  "gene_symbol": "ILRUN",
  "gene_name": "Protein ILRUN",
  "term_label": "phagophore assembly site",
  "term_id": "GO:0000407"
}